myosin XIII complex [GO:0031483] (cellular component) Definition: A myosin complex containing one or more class XIII myosin heavy chains and associated light chains. Relationships: is a type of unconventional myosin complex [GO:0016461] References: PMID:10722873